{
  "term_label": "N-acylphosphatidylethanolamine metabolic process",
  "gene_name": "Phospholipase A and acyltransferase 3",
  "gene_symbol": "PLAAT3",
  "gene": "UniProtKB:P53816",
  "term_id": "GO:0070292"
}